{
  "term_id": "UNKNOWN:0001",
  "gene_name": "Protein shisa-9",
  "term_label": "Unknown molecular function",
  "gene_symbol": "SHISA9",
  "gene": "UniProtKB:B4DS77"
}